cellular response to vitamin K [GO:0071307] (biological process) Definition: Any process that results in a change in state or activity of a cell (in terms of movement, secretion, enzyme production, gene expression, etc.) as a result of a vitamin K stimulus. Sources: GOC:mah Relationships: is a type of response to vitamin K [GO:0032571]; is a type of cellular response to vitamin [GO:0071295]; is a type of GO:1901655 Subtypes: cellular response to menadione [GO:0036245], GO:0071308, GO:0071309